floral organ structural organization [GO:0048450] (biological process) Sources: GOC:PO_curators, GOC:jid, PO:0025395 Subtypes: petal structural organization [GO:0048452], sepal structural organization [GO:0048454], stamen structural organization [GO:0048456], GO:0048463 Relationships: is a type of GO:0048444; is_a GO:0048532; is part of flower structural organization [GO:0048461] Definition: The process that contributes to the act of creating the structural organization of floral organs. This process pertains to the physical shaping of a rudimentary structure. Also known as: floral organ structural organisation